{
  "gene_name": "Leukemia inhibitory factor",
  "term_label": "growth factor activity",
  "gene_symbol": "LIF",
  "term_id": "GO:0008083",
  "gene": "UniProtKB:P15018"
}